{
  "gene_name": "Nucleolar pre-ribosomal-associated protein 1",
  "gene": "UniProtKB:O60287",
  "term_label": "maturation of LSU-rRNA from tricistronic rRNA transcript (SSU-rRNA, 5.8S rRNA, LSU-rRNA)",
  "term_id": "GO:0000463",
  "gene_symbol": "URB1"
}